{
  "gene_name": "Calretinin",
  "gene": "UniProtKB:P22676",
  "term_label": "cytosol",
  "term_id": "GO:0005829",
  "gene_symbol": "CALB2"
}